{
  "gene_name": "Breakpoint cluster region protein",
  "term_id": "GO:0016020",
  "gene": "UniProtKB:P11274",
  "term_label": "membrane",
  "gene_symbol": "BCR"
}